{
  "gene_symbol": "PRNT",
  "term_label": "Unknown cellular component",
  "term_id": "UNKNOWN:0003",
  "gene_name": "Putative testis-specific prion protein",
  "gene": "UniProtKB:Q86SH4"
}